{
  "term_id": "GO:0006355",
  "term_label": "regulation of DNA-templated transcription",
  "gene_name": "Zinc finger protein 738",
  "gene": "UniProtKB:Q8NE65",
  "gene_symbol": "ZNF738"
}